{
  "gene_symbol": "OCRL",
  "gene": "UniProtKB:Q01968",
  "gene_name": "Inositol polyphosphate 5-phosphatase OCRL",
  "term_label": "neuron projection",
  "term_id": "GO:0043005"
}